{
  "gene": "UniProtKB:Q8NFW9",
  "gene_symbol": "MYRIP",
  "term_id": "UNKNOWN:0002",
  "gene_name": "Rab effector MyRIP",
  "term_label": "Unknown biological process"
}